{
  "gene": "UniProtKB:Q8NFP4",
  "gene_symbol": "MDGA1",
  "gene_name": "MAM domain-containing glycosylphosphatidylinositol anchor protein 1",
  "term_label": "nervous system development",
  "term_id": "GO:0007399"
}